4-hydroxybutyrate CoA-transferase activity [GO:0008411] (MF) Definition: Catalysis of the transfer of a coenzyme A (CoA) group to 4-hydroxybutyrate. Relationships: is a type of CoA-transferase activity [GO:0008410] References: PMID:25452282 Sources: GOC:jl